{
  "gene_symbol": "SNX13",
  "term_label": "Unknown biological process",
  "gene_name": "Sorting nexin-13",
  "gene": "UniProtKB:Q9Y5W8",
  "term_id": "UNKNOWN:0002"
}